{
  "gene": "UniProtKB:Q53FT3",
  "term_label": "nuclear import signal receptor activity",
  "gene_name": "Protein Hikeshi",
  "gene_symbol": "HIKESHI",
  "term_id": "GO:0061608"
}